{
  "term_label": "chromatin remodeling",
  "gene_name": "Host cell factor 1",
  "term_id": "GO:0006338",
  "gene_symbol": "HCFC1",
  "gene": "UniProtKB:P51610"
}